L-hydroxyproline transmembrane transporter activity [GO:0034590] (molecular function) Relationships: is a type of monocarboxylic acid transmembrane transporter activity [GO:0008028]; is a type of GO:0015179; is a type of modified amino acid transmembrane transporter activity [GO:0072349]; is part of GO:0034589 Definition: Enables the transfer of L-hydroxyproline from one side of a membrane to the other. Also known as: 4-hydroxyproline transmembrane transporter activity References: PMID:14502423 Sources: GOC:mah